{
  "gene": "UniProtKB:Q7Z2Z1",
  "gene_name": "Treslin",
  "term_id": "GO:0033314",
  "term_label": "mitotic DNA replication checkpoint signaling",
  "gene_symbol": "TICRR"
}